regulation of innate immunity memory response [GO:1905680] (biological process) Sources: GOC:TermGenie, GO_REF:0000058 Definition: Any process that modulates the frequency, rate or extent of innate immunity memory response. Relationships: is a type of regulation of innate immune response [GO:0045088]; regulates innate immunity memory response [GO:0090714] Subtypes: negative regulation of innate immunity memory response [GO:1905681], positive regulation of innate immunity memory response [GO:1905682]